{
  "term_id": "GO:0000122",
  "gene_symbol": "KANK2",
  "term_label": "negative regulation of transcription by RNA polymerase II",
  "gene_name": "KN motif and ankyrin repeat domain-containing protein 2",
  "gene": "UniProtKB:Q63ZY3"
}